{
  "term_label": "endoplasmic reticulum-Golgi intermediate compartment",
  "gene": "UniProtKB:Q9UBF2",
  "term_id": "GO:0005793",
  "gene_symbol": "COPG2",
  "gene_name": "Coatomer subunit gamma-2"
}